T cell tolerance induction [GO:0002517] (biological process) Subtypes: GO:0002458, central T cell tolerance induction [GO:0002512], T cell anergy [GO:0002870] Regulation: regulated by regulation of T cell tolerance induction [GO:0002664]; negatively regulated by negative regulation of T cell tolerance induction [GO:0002665]; positively regulated by GO:0002666 Also known as: T lymphocyte tolerance induction, T-cell tolerance induction, T-lymphocyte tolerance induction Definition: A process involving any mechanism for tolerance induction in T cells. Relationships: is a type of tolerance induction [GO:0002507] References: PMID:16551263 Sources: GOC:jal, ISBN:0781735149